{
  "term_id": "GO:0000122",
  "gene": "UniProtKB:Q8N7X4",
  "gene_symbol": "MAGEB6",
  "gene_name": "Melanoma-associated antigen B6",
  "term_label": "negative regulation of transcription by RNA polymerase II"
}